{
  "term_label": "cilium assembly",
  "gene_name": "Thioredoxin domain-containing protein 3",
  "term_id": "GO:0060271",
  "gene_symbol": "NME8",
  "gene": "UniProtKB:Q8N427"
}